{
  "gene": "UniProtKB:Q7Z5J8",
  "term_id": "UNKNOWN:0001",
  "gene_symbol": "ANKAR",
  "term_label": "Unknown molecular function",
  "gene_name": "Ankyrin and armadillo repeat-containing protein"
}